{
  "gene": "UniProtKB:P33151",
  "gene_symbol": "CDH5",
  "term_id": "GO:0005923",
  "term_label": "bicellular tight junction",
  "gene_name": "Cadherin-5"
}